protein quality control for misfolded or incompletely synthesized proteins [GO:0006515] (biological process) Relationships: is a type of proteolysis involved in protein catabolic process [GO:0051603] Subtypes: GO:0071630, cytoplasm protein quality control [GO:0140455], mitochondrial protein quality control [GO:0141164] Sources: GOC:jl Also known as: protein quality control by the ubiquitin-proteasome system, degradation of misfolded or incompletely synthesized proteins, misfolded or incompletely synthesized protein breakdown, misfolded or incompletely synthesized protein catabolic process, misfolded or incompletely synthesized protein catabolism, misfolded or incompletely synthesized protein degradation, protein quality control (PQC) Definition: The chemical reactions and pathways resulting in the breakdown of misfolded or attenuated proteins.